prenyl-diphosphatase activity [GO:0050210] (MF) Also known as: prenyl-pyrophosphatase activity, prenol pyrophosphatase activity, prenyl-diphosphate diphosphohydrolase activity, prenylphosphatase activity Sources: RHEA:21496 Relationships: is a type of GO:0016794 Definition: Catalysis of the reaction: dimethylallyl diphosphate + H2O = diphosphate + prenol.